{
  "gene_symbol": "TMED2",
  "term_label": "endoplasmic reticulum",
  "gene_name": "Transmembrane emp24 domain-containing protein 2",
  "term_id": "GO:0005783",
  "gene": "UniProtKB:Q15363"
}